TOR complex [GO:0038201] (cellular component) Definition: A protein complex that contains at least TOR (target of rapamycin) in complex with other signaling components. Mediates the phosphorylation and activation of downstream signaling components including PKB (AKT) or S6K. Sources: Wikipedia:MTORC1, Wikipedia:MTORC2 Also known as: TOR signaling complex, target of rapamycin complex, mTOR complex Relationships: is a type of intracellular protein-containing complex [GO:0140535] Subtypes: TORC1 complex [GO:0031931], TORC2 complex [GO:0031932]